{
  "term_label": "Unknown biological process",
  "gene_symbol": "SEC14L2",
  "gene_name": "SEC14-like protein 2",
  "gene": "UniProtKB:O76054",
  "term_id": "UNKNOWN:0002"
}